regulation of membrane lipid metabolic process [GO:1905038] (biological process) Definition: Any process that modulates the frequency, rate or extent of membrane lipid metabolic process. Subtypes: regulation of sphingolipid biosynthetic process [GO:0090153], regulation of glucosylceramide catabolic process [GO:2000752], regulation of sphingomyelin catabolic process [GO:2000754] Also known as: regulation of membrane lipid metabolism Relationships: is a type of regulation of lipid metabolic process [GO:0019216]; regulates membrane lipid metabolic process [GO:0006643] References: PMID:25954280 Sources: GOC:TermGenie, GO_REF:0000058